regulation of cardiac myofibril assembly [GO:1905304] (biological process) Relationships: is a type of regulation of cell development [GO:0060284]; is a type of regulation of actomyosin structure organization [GO:0110020]; is a type of GO:1902115; is a type of regulation of supramolecular fiber organization [GO:1902903]; regulates GO:0055003 Also known as: regulation of cardiac myofibril development, regulation of cardiac myofibril morphogenesis, regulation of heart myofibril assembly References: PMID:16151019 Sources: GOC:BHF, GOC:TermGenie, GOC:rl, GO_REF:0000058 Subtypes: negative regulation of cardiac myofibril assembly [GO:1905305], positive regulation of cardiac myofibril assembly [GO:1905306] Definition: Any process that modulates the frequency, rate or extent of cardiac myofibril assembly.